{
  "gene_symbol": "STX5",
  "term_id": "GO:0006886",
  "gene": "UniProtKB:Q13190",
  "gene_name": "Syntaxin-5",
  "term_label": "intracellular protein transport"
}